negative regulation of neuron differentiation [GO:0045665] (BP) Definition: Any process that stops, prevents, or reduces the frequency, rate or extent of neuron differentiation. Relationships: is a type of negative regulation of cell differentiation [GO:0045596]; is a type of GO:0045664; negatively regulates GO:0030182 Also known as: down regulation of neuron differentiation, down-regulation of neuron differentiation, downregulation of neuron differentiation, inhibition of neuron differentiation Subtypes: negative regulation of mechanoreceptor differentiation [GO:0045632], negative regulation of photoreceptor cell differentiation [GO:0046533], negative regulation of stomach neuroendocrine cell differentiation [GO:0061106], GO:0120007, GO:1902830, GO:1902870, negative regulation of dopaminergic neuron differentiation [GO:1904339], negative regulation of cerebellar neuron development [GO:1905080], negative regulation of forebrain neuron differentiation [GO:2000978] Sources: GOC:go_curators